{
  "term_id": "GO:0006357",
  "gene_symbol": "ZNF75CP",
  "gene_name": "Putative zinc finger protein 75C",
  "term_label": "regulation of transcription by RNA polymerase II",
  "gene": "UniProtKB:Q92670"
}